{
  "gene": "UniProtKB:Q06136",
  "term_label": "sphingolipid biosynthetic process",
  "gene_name": "3-ketodihydrosphingosine reductase",
  "gene_symbol": "KDSR",
  "term_id": "GO:0030148"
}